RNA strand-exchange activity [GO:0034057] (molecular function) References: PMID:9769100 Sources: GOC:mcc Definition: Facilitates the displacement of one strand of an RNA-RNA duplex and its replacement with a different strand of higher complementarity. Relationships: is a type of double-stranded RNA binding [GO:0003725]; is a type of single-stranded RNA binding [GO:0003727]